{
  "term_label": "cytoplasm",
  "gene": "UniProtKB:Q8IV48",
  "gene_symbol": "ERI1",
  "term_id": "GO:0005737",
  "gene_name": "3'-5' exoribonuclease 1"
}